misfolded RNA binding [GO:0034336] (molecular function) Also known as: RNA chaperone References: PMID:10393192 Sources: GOC:mah Definition: Binding to an RNA molecule that has assumed an incorrect conformation. Relationships: is a type of RNA binding [GO:0003723]